{
  "term_label": "Unknown molecular function",
  "gene_symbol": "DLEU7",
  "term_id": "UNKNOWN:0001",
  "gene_name": "Leukemia-associated protein 7",
  "gene": "UniProtKB:Q6UYE1"
}